{
  "term_label": "endoplasmic reticulum membrane",
  "term_id": "GO:0005789",
  "gene_name": "Phosphatidylinositol-glycan biosynthesis class F protein",
  "gene_symbol": "PIGF",
  "gene": "UniProtKB:Q07326"
}